{
  "gene_symbol": "FBXL19-AS1",
  "term_label": "Unknown cellular component",
  "term_id": "UNKNOWN:0003",
  "gene_name": "Putative uncharacterized protein FBXL19-AS1",
  "gene": "UniProtKB:Q494R0"
}